acetate kinase (diphosphate) activity [GO:0047601] (molecular function) Also known as: acetate kinase (pyrophosphate) activity, diphosphate:acetate phosphotransferase activity, pyrophosphate-acetate phosphotransferase activity Definition: Catalysis of the reaction: acetate + diphosphate = acetyl phosphate + phosphate. Relationships: is a type of GO:0016301; is a type of GO:0016774 Sources: EC:2.7.2.12, RHEA:24276